{
  "gene_name": "Inner centromere protein",
  "gene_symbol": "INCENP",
  "term_id": "GO:0030496",
  "term_label": "midbody",
  "gene": "UniProtKB:Q9NQS7"
}